{
  "gene_symbol": "FLNA",
  "gene_name": "Filamin-A",
  "term_label": "Unknown cellular component",
  "gene": "UniProtKB:P21333",
  "term_id": "UNKNOWN:0003"
}